{
  "term_label": "mitotic spindle organization",
  "gene": "UniProtKB:Q496M5",
  "gene_symbol": "PLK5",
  "term_id": "GO:0007052",
  "gene_name": "Inactive serine_threonine-protein kinase PLK5"
}